{
  "term_id": "GO:0008009",
  "term_label": "chemokine activity",
  "gene": "UniProtKB:Q8NHW4",
  "gene_symbol": "CCL4L1",
  "gene_name": "C-C motif chemokine 4-like"
}